{
  "term_label": "extracellular space",
  "gene": "UniProtKB:Q08830",
  "term_id": "GO:0005615",
  "gene_symbol": "FGL1",
  "gene_name": "Fibrinogen-like protein 1"
}